mast cell mediated immunity [GO:0002448] (biological process) Definition: Any process involved in the carrying out of an immune response by a mast cell. Sources: GOC:add, GO_REF:0000022, ISBN:0781735149 Relationships: is a type of myeloid leukocyte mediated immunity [GO:0002444] Subtypes: type I hypersensitivity mediated by mast cells [GO:0002558]